cysteine-type deubiquitinase activity [GO:0004843] (molecular function) Definition: An thiol-dependent isopeptidase activity that cleaves ubiquitin from a target protein to which it is conjugated. References: PMID:30783221 Sources: GOC:jh2 Also known as: deubiquitinase, deubiquitinase activity, deubiquitinating enzyme, deubiquitylase, ubiquitin hydrolase activity, ubiquitin-specific protease activity, ubiquitinyl hydrolase activity, thiol-dependent deubiquitinase, thiol-dependent ubiquitin-specific protease activity, thiol-dependent ubiquitinyl hydrolase activity, UBP, UCH2, ubiquitinyl hydrolase 1 activity, ubiquitin C-terminal hydrolase Relationships: is a type of cysteine-type peptidase activity [GO:0008234]; is a type of deubiquitinase activity [GO:0101005] Subtypes: Met1-linked polyubiquitin deubiquitinase activity [GO:0061815] Regulation: positively regulated by GO:2000158